{
  "gene_name": "Thyroid transcription factor 1-associated protein 26",
  "gene_symbol": "CCDC59",
  "term_id": "UNKNOWN:0002",
  "term_label": "Unknown biological process",
  "gene": "UniProtKB:Q9P031"
}